positive regulation of platelet-derived growth factor receptor-alpha signaling pathway [GO:2000585] (biological process) Relationships: is a type of positive regulation of platelet-derived growth factor receptor signaling pathway [GO:0010641]; is a type of regulation of platelet-derived growth factor receptor-alpha signaling pathway [GO:2000583]; positively regulates GO:0035790 Definition: Any process that activates or increases the frequency, rate or extent of platelet-derived growth factor receptor-alpha signaling pathway. Also known as: positive regulation of PDGF receptor-alpha signaling pathway, positive regulation of alphaPDGF receptor signaling pathway, positive regulation of platelet-derived growth factor receptor-alpha signalling pathway, positive regulation of PDGFR-alpha signaling pathway Sources: GOC:obol